{
  "term_label": "Unknown biological process",
  "gene_symbol": "CCDC192",
  "gene_name": "Coiled-coil domain-containing protein 192",
  "gene": "UniProtKB:P0DO97",
  "term_id": "UNKNOWN:0002"
}